{
  "gene": "UniProtKB:Q2KJY2",
  "gene_symbol": "KIF26B",
  "term_id": "UNKNOWN:0003",
  "term_label": "Unknown cellular component",
  "gene_name": "Kinesin-like protein KIF26B"
}